{
  "term_id": "GO:0005737",
  "gene_name": "Kynureninase",
  "term_label": "cytoplasm",
  "gene_symbol": "KYNU",
  "gene": "UniProtKB:Q16719"
}